positive regulation of epidermal cell differentiation [GO:0045606] (biological process) Also known as: up regulation of epidermal cell differentiation, up-regulation of epidermal cell differentiation, upregulation of epidermal cell differentiation, activation of epidermal cell differentiation, stimulation of epidermal cell differentiation, positive regulation of hypodermal cell differentiation Sources: GOC:go_curators Definition: Any process that activates or increases the frequency, rate or extent of epidermal cell differentiation. Subtypes: positive regulation of inner ear auditory receptor cell differentiation [GO:0045609], positive regulation of keratinocyte differentiation [GO:0045618] Relationships: is a type of positive regulation of epithelial cell differentiation [GO:0030858]; is a type of regulation of epidermal cell differentiation [GO:0045604]; is a type of positive regulation of epidermis development [GO:0045684]; positively regulates GO:0009913